{
  "term_label": "nucleus",
  "gene_symbol": "USP17L4",
  "gene_name": "Inactive ubiquitin carboxyl-terminal hydrolase 17-like protein 4",
  "term_id": "GO:0005634",
  "gene": "UniProtKB:A6NCW7"
}